{
  "term_label": "fructose-6-phosphate binding",
  "gene_symbol": "GCKR",
  "gene_name": "Glucokinase regulatory protein",
  "term_id": "GO:0070095",
  "gene": "UniProtKB:Q14397"
}